tRNA-type intron splice site recognition and cleavage [GO:0000379] (biological process) Relationships: is a type of GO:0006396; is part of tRNA splicing, via endonucleolytic cleavage and ligation [GO:0006388] Definition: RNA processing that begins when the tertiary structure of a tRNA type intron is recognized, and ends when the endonucleolytic cleavage of the RNA at both the 5' and 3' splice sites occurs. Sources: GOC:krc, GOC:mah, ISBN:0879695897